chromosome attachment to the nuclear envelope [GO:0097240] (biological process) Definition: The process in which chromatin is anchored to the nuclear envelope. References: PMID:31635174 Sources: GOC:vw Relationships: is a type of cell cycle process [GO:0022402]; is_a GO:0050000 Also known as: attachment of chromatin to nuclear envelope Subtypes: meiotic attachment of telomere to nuclear envelope [GO:0070197], centromere clustering at the mitotic interphase nuclear envelope [GO:0072766], subnuclear spatial organization of silent mating-type cassette heterochromatin [GO:0140464], attachment of telomeric heterochromatin to nuclear envelope [GO:0140698], DNA double-strand break attachment to nuclear envelope [GO:1990683] Regulation: RO_0002211 by regulation of chromosome attachment to the nuclear envelope [GO:0120264]; negatively regulated by negative regulation of chromosome attachment to the nuclear envelope [GO:0120265]; positively regulated by GO:0120266